{
  "term_label": "intracellular protein transport",
  "gene": "UniProtKB:Q4ADV7",
  "gene_symbol": "RIC1",
  "gene_name": "Guanine nucleotide exchange factor subunit RIC1",
  "term_id": "GO:0006886"
}